inhibitory G protein-coupled receptor phosphorylation [GO:0002030] (biological process) Also known as: inhibitory G-protein coupled receptor phosphorylation Regulation: RO_0002211 by regulation of inhibitory G protein-coupled receptor phosphorylation [GO:1904323]; negatively regulated by GO:1904324; positively regulated by GO:1904325 References: PMID:8396717 Relationships: is a type of protein phosphorylation [GO:0006468]; is part of desensitization of G protein-coupled receptor signaling pathway [GO:0002029] Definition: The process that inhibits the signaling function of a G protein-coupled receptor by addition of a phosphate group to its third intracellular loop consensus site.